hyaluranon cable assembly [GO:0036118] (biological process) Also known as: HA cable assembly Relationships: is_a cellular component assembly [GO:0022607] Definition: A process that results in the aggregation, arrangement and bonding together of a hyaluranon cable, a cable structure, surrounding some cell types (e.g. proximal or bronchial tubular epithelial cells), and composed of hyaluranon (HA), a ubiquitous connective tissue glycosaminoglycan. References: PMID:16900089 Sources: GOC:yaf Regulation: regulated by regulation of hyaluranon cable assembly [GO:1900104]; negatively regulated by negative regulation of hyaluranon cable assembly [GO:1900105]; positively regulated by positive regulation of hyaluranon cable assembly [GO:1900106]